{
  "term_id": "UNKNOWN:0001",
  "term_label": "Unknown molecular function",
  "gene_name": "Uncharacterized protein KRT10-AS1",
  "gene_symbol": "KRT10-AS1",
  "gene": "UniProtKB:Q8N816"
}